{
  "gene_name": "Alpha-actinin-4",
  "term_label": "cell junction",
  "gene": "UniProtKB:O43707",
  "gene_symbol": "ACTN4",
  "term_id": "GO:0030054"
}